gastric inhibitory peptide receptor activity [GO:0016519] (molecular function) Definition: Combining with gastric inhibitory peptide (GIP) and transmitting the signal across the membrane to activate an associated G-protein. References: PMID:8243312 Sources: GOC:mah Also known as: GIP receptor activity, glucose-dependent insulinotropic polypeptide receptor activity Relationships: is a type of GO:0004930; is part of gastric inhibitory peptide signaling pathway [GO:0038192]